{
  "gene_symbol": "DIMT1",
  "term_id": "GO:0005730",
  "gene": "UniProtKB:Q9UNQ2",
  "gene_name": "Probable dimethyladenosine transferase",
  "term_label": "nucleolus"
}